{
  "gene_name": "CUGBP Elav-like family member 1",
  "gene": "UniProtKB:Q92879",
  "term_label": "regulation of alternative mRNA splicing, via spliceosome",
  "term_id": "GO:0000381",
  "gene_symbol": "CELF1"
}